{
  "term_id": "UNKNOWN:0003",
  "gene": "UniProtKB:P0C7W8",
  "term_label": "Unknown cellular component",
  "gene_symbol": "FAM90A13P",
  "gene_name": "Putative protein FAM90A13P"
}